{
  "term_label": "neuron differentiation",
  "gene_name": "Protein Wnt-2",
  "gene": "UniProtKB:P09544",
  "term_id": "GO:0030182",
  "gene_symbol": "WNT2"
}